m-xylene catabolic process [GO:0042185] (BP) Also known as: m-xylene breakdown, m-xylene catabolism, m-xylene degradation, meta-xylene catabolic process, meta-xylene catabolism Definition: The chemical reactions and pathways resulting in the breakdown of m-xylene, 1,3-dimethylbenzene, a colorless, liquid aromatic hydrocarbon. Relationships: is a type of xylene catabolic process [GO:0042184] Sources: GOC:go_curators, GOC:jl